{
  "term_id": "UNKNOWN:0003",
  "term_label": "Unknown cellular component",
  "gene_name": "Receptor-type tyrosine-protein phosphatase mu",
  "gene_symbol": "PTPRM",
  "gene": "UniProtKB:P28827"
}